{
  "gene": "UniProtKB:A0A1B0GX95",
  "gene_name": "T cell receptor beta variable 7-4",
  "term_id": "GO:0005886",
  "gene_symbol": "TRBV7-4",
  "term_label": "plasma membrane"
}